{
  "term_label": "Unknown biological process",
  "gene_symbol": "NDUFA8",
  "gene_name": "NADH dehydrogenase [ubiquinone] 1 alpha subcomplex subunit 8",
  "term_id": "UNKNOWN:0002",
  "gene": "UniProtKB:P51970"
}